{
  "gene_name": "Carbonic anhydrase 2",
  "gene": "UniProtKB:P00918",
  "term_label": "cytoplasm",
  "term_id": "GO:0005737",
  "gene_symbol": "CA2"
}